negative regulation of c-di-GMP signaling [GO:0061942] (biological process) References: PMID:22864416 Relationships: is a type of GO:0010648; is a type of GO:0023057; is a type of regulation of c-di-GMP signaling [GO:0061940]; negatively regulates c-di-GMP signaling [GO:0061939] Definition: Any process that decreases the rate, frequency or extent of c-di-GMP signaling.